{
  "term_id": "UNKNOWN:0003",
  "term_label": "Unknown cellular component",
  "gene_name": "L-fucose kinase",
  "gene": "UniProtKB:Q8N0W3",
  "gene_symbol": "FCSK"
}